{
  "term_id": "UNKNOWN:0001",
  "gene_name": "Mitoguardin 2",
  "term_label": "Unknown molecular function",
  "gene_symbol": "MIGA2",
  "gene": "UniProtKB:Q7L4E1"
}